{
  "gene_symbol": "ADAM17",
  "gene": "UniProtKB:P78536",
  "term_label": "plasma membrane",
  "term_id": "GO:0005886",
  "gene_name": "Disintegrin and metalloproteinase domain-containing protein 17"
}